{
  "gene_name": "BTB_POZ domain-containing adapter for CUL3-mediated RhoA degradation protein 3",
  "gene": "UniProtKB:Q9H3F6",
  "gene_symbol": "KCTD10",
  "term_id": "GO:0043161",
  "term_label": "proteasome-mediated ubiquitin-dependent protein catabolic process"
}